{
  "gene": "UniProtKB:O75409",
  "term_id": "GO:0031507",
  "gene_name": "Huntingtin-interacting protein M",
  "term_label": "heterochromatin formation",
  "gene_symbol": "H2AP"
}